cell migration involved in mesendoderm migration [GO:0090134] (biological process) Definition: The orderly movement of epithelial cells from one site to another that contributes to the migration of mesendodermal tissue. Relationships: is a type of cell migration involved in gastrulation [GO:0042074]; is part of mesendoderm migration [GO:0090133] Sources: GOC:ascb_2009, GOC:dph, GOC:tb